{
  "term_id": "UNKNOWN:0003",
  "gene_name": "Zinc finger matrin-type protein 3",
  "term_label": "Unknown cellular component",
  "gene_symbol": "ZMAT3",
  "gene": "UniProtKB:Q9HA38"
}